{
  "term_label": "serine-type endopeptidase activity",
  "gene_symbol": "HGFAC",
  "gene_name": "Hepatocyte growth factor activator",
  "gene": "UniProtKB:Q04756",
  "term_id": "GO:0004252"
}